fibrinogen complex [GO:0005577] (CC) Sources: ISBN:0198547684 Also known as: fibrinogen, fibrinogen alpha chain, fibrinogen beta chain, fibrinogen gamma chain Relationships: is a type of GO:0032991; is part of GO:0005615 Definition: A highly soluble, elongated protein complex found in blood plasma and involved in clot formation. It is converted into fibrin monomer by the action of thrombin. In the mouse, fibrinogen is a hexamer, 46 nm long and 9 nm maximal diameter, containing two sets of nonidentical chains (alpha, beta, and gamma) linked together by disulfide bonds.